{
  "term_label": "Unknown molecular function",
  "gene_name": "Small integral membrane protein 8",
  "gene_symbol": "SMIM8",
  "gene": "UniProtKB:Q96KF7",
  "term_id": "UNKNOWN:0001"
}